{
  "term_id": "GO:0005634",
  "gene_name": "Metallothionein-3",
  "gene": "UniProtKB:P25713",
  "term_label": "nucleus",
  "gene_symbol": "MT3"
}